{
  "term_id": "GO:0005737",
  "gene_name": "Sterile alpha motif domain-containing protein 9-like",
  "term_label": "cytoplasm",
  "gene_symbol": "SAMD9L",
  "gene": "UniProtKB:Q8IVG5"
}